epiboly involved in wound healing [GO:0090505] (biological process) Definition: The expansion of one cell sheet over other cells involved in wound healing. Sources: GOC:dph, GOC:tb Relationships: is a type of epiboly [GO:0090504]; is part of wound healing [GO:0042060]